{
  "term_label": "lipid droplet",
  "gene": "UniProtKB:Q8IZV5",
  "gene_symbol": "RDH10",
  "gene_name": "Retinol dehydrogenase 10",
  "term_id": "GO:0005811"
}